{
  "gene_name": "Ribosomal protein eL39-like 2",
  "term_id": "GO:0007283",
  "gene": "UniProtKB:Q96EH5",
  "term_label": "spermatogenesis",
  "gene_symbol": "RPL39L"
}